{
  "term_label": "Unknown biological process",
  "gene": "UniProtKB:Q9Y2E5",
  "term_id": "UNKNOWN:0002",
  "gene_name": "Epididymis-specific alpha-mannosidase",
  "gene_symbol": "MAN2B2"
}